purine ribonucleoside binding [GO:0032550] (molecular function) Definition: Binding to a purine ribonucleoside, a compound consisting of a purine base linked to ribose. Sources: GOC:mah Subtypes: guanosine binding [GO:1905108] Relationships: is a type of purine nucleoside binding [GO:0001883]; is a type of ribonucleoside binding [GO:0032549]